regulation of systemic arterial blood pressure by aortic body chemoreceptor signaling [GO:0003028] (biological process) Sources: GOC:dph, GOC:mtg_cardio, GOC:tb Relationships: is_a regulation of systemic arterial blood pressure by chemoreceptor signaling [GO:0001979] Definition: The process that modulates blood pressure by the action of chemoreceptors found in the aortic bodies and their resultant modulation of the vasomotor center. Chemoreceptors respond to oxygen, carbon dioxide and hydrogen ions. Also known as: aortic body chemoreceptor regulation of systemic arterial blood pressure, aortic body chemoreceptor response to lowering of systemic arterial blood pressure, regulation of systemic arterial blood pressure by aortic body chemoreceptor signalling